{
  "gene_name": "H(+)_Cl(-) exchange transporter 6",
  "term_label": "chloride transport",
  "gene_symbol": "CLCN6",
  "term_id": "GO:0006821",
  "gene": "UniProtKB:P51797"
}